{
  "gene_symbol": "GMEB1",
  "term_id": "GO:0006357",
  "gene": "UniProtKB:Q9Y692",
  "term_label": "regulation of transcription by RNA polymerase II",
  "gene_name": "Glucocorticoid modulatory element-binding protein 1"
}